immunoglobulin light chain V-J recombination [GO:0071708] (biological process) Sources: GOC:add, ISBN:0781735149 Relationships: is a type of immunoglobulin V(D)J recombination [GO:0033152] Definition: The process in which immunoglobulin light chain V and J gene segments are recombined within a single locus utilizing the conserved heptamer and nonomer recombination signal sequences (RSS). Also known as: immunoglobulin V(D)J joining, immunoglobulin V(D)J recombination, immunoglobulin V-J joining